{
  "gene_symbol": "KRT26",
  "gene_name": "Keratin, type I cytoskeletal 26",
  "term_label": "structural constituent of skin epidermis",
  "gene": "UniProtKB:Q7Z3Y9",
  "term_id": "GO:0030280"
}